germ tube septin ring [GO:0032172] (cellular component) Definition: A tight ring-shaped structure that forms in the division plane within the germ tube of filamentous fungi at sites where a septum will form; composed of septins as well as septin-associated proteins. References: PMID:16151244 Sources: GOC:krc Relationships: is a type of septin ring [GO:0005940]; is part of GO:0032179